{
  "gene": "UniProtKB:Q96KC9",
  "term_label": "motile cilium",
  "gene_symbol": "CABS1",
  "gene_name": "Calcium-binding and spermatid-specific protein 1",
  "term_id": "GO:0031514"
}